regulation of anoikis [GO:2000209] (biological process) Definition: Any process that modulates the frequency, rate or extent of anoikis. Sources: GOC:mah Also known as: regulation of detachment induced cell death, regulation of suspension induced apoptosis Relationships: is a type of regulation of apoptotic process [GO:0042981]; regulates anoikis [GO:0043276] Subtypes: positive regulation of anoikis [GO:2000210], GO:2000811